lipid X metabolic process [GO:2001289] (biological process) Also known as: 2-deoxy-3-O-[(3R)-3-hydroxytetradecanoyl]-2-{[(3R)-3-hydroxytetradecanoyl]amino}-1-O-phosphono-alpha-D-glucopyranose metabolic process, 2-deoxy-3-O-[(3R)-3-hydroxytetradecanoyl]-2-{[(3R)-3-hydroxytetradecanoyl]amino}-1-O-phosphono-alpha-D-glucopyranose metabolism, lipid X metabolism, 2,3-Bis(3-hydroxytetradecanoyl)-beta-D-glucosaminyl 1-phosphate metabolic process, 2,3-Bis(3-hydroxytetradecanoyl)-beta-D-glucosaminyl 1-phosphate metabolism, 2,3-Bis(beta-hydoroxymyristoyl)-beta-D-glucosaminyl 1-phosphate metabolic process, 2,3-Bis(beta-hydoroxymyristoyl)-beta-D-glucosaminyl 1-phosphate metabolism Relationships: is a type of GO:0006040; is a type of GO:0006796; is a type of organophosphate metabolic process [GO:0019637] Sources: GOC:obol Definition: The chemical reactions and pathways involving lipid X, 2,3-diacylglucosamine 1-phosphate.